{
  "term_label": "Unknown molecular function",
  "term_id": "UNKNOWN:0001",
  "gene_name": "INO80 complex subunit B",
  "gene_symbol": "INO80B",
  "gene": "UniProtKB:Q9C086"
}